{
  "gene": "UniProtKB:P22310",
  "gene_name": "UDP-glucuronosyltransferase 1A4",
  "term_label": "estrogen metabolic process",
  "gene_symbol": "UGT1A4",
  "term_id": "GO:0008210"
}